{
  "term_label": "nucleus",
  "gene_symbol": "MCM9",
  "gene": "UniProtKB:Q9NXL9",
  "gene_name": "DNA helicase MCM9",
  "term_id": "GO:0005634"
}